{
  "term_id": "GO:0005768",
  "gene": "UniProtKB:Q8WUM4",
  "gene_name": "Programmed cell death 6-interacting protein",
  "gene_symbol": "PDCD6IP",
  "term_label": "endosome"
}